{
  "gene_symbol": "CFAP97",
  "gene_name": "Cilia- and flagella-associated protein 97",
  "term_label": "Unknown molecular function",
  "gene": "UniProtKB:Q9P2B7",
  "term_id": "UNKNOWN:0001"
}